{
  "gene": "UniProtKB:Q9NX05",
  "gene_symbol": "FAM120C",
  "gene_name": "Constitutive coactivator of PPAR-gamma-like protein 2",
  "term_label": "Unknown molecular function",
  "term_id": "UNKNOWN:0001"
}